symbiont-mediated disruption of host cell PML body [GO:0075342] (biological process) Definition: The process in which an organism effects a change that impairs the structure or function of the host PML body. A PML body is a nuclear body that reacts against SP100 auto-antibodies (PML = promyelocytic leukemia). The host is defined as the larger of the organisms involved in a symbiotic interaction. Also known as: catabolism by symbiont of host cell PML body, degradation by symbiont of host cell PML body, disassembly by symbiont of host cell PML NB, disassembly by symbiont of host cell PML body, disassembly by symbiont of host cell PML body during symbiotic interaction, disassembly by symbiont of host cell PML nuclear body, disruption by symbiont of host cell PML body Sources: GOC:BHF, GOC:jl Relationships: is a type of symbiont-mediated disruption of host cellular anatomical structure [GO:0052008]